{
  "gene_name": "Patatin-like phospholipase domain-containing protein 2",
  "term_label": "membrane",
  "gene": "UniProtKB:Q96AD5",
  "term_id": "GO:0016020",
  "gene_symbol": "PNPLA2"
}